{
  "term_label": "external side of plasma membrane",
  "gene": "UniProtKB:Q7Z7D3",
  "gene_symbol": "VTCN1",
  "term_id": "GO:0009897",
  "gene_name": "V-set domain-containing T-cell activation inhibitor 1"
}